{
  "term_id": "GO:0000978",
  "gene": "UniProtKB:Q9UPW6",
  "gene_symbol": "SATB2",
  "term_label": "RNA polymerase II cis-regulatory region sequence-specific DNA binding",
  "gene_name": "DNA-binding protein SATB2"
}